{
  "term_id": "UNKNOWN:0003",
  "term_label": "Unknown cellular component",
  "gene_symbol": "PTX4",
  "gene_name": "Pentraxin-4",
  "gene": "UniProtKB:Q96A99"
}